{
  "gene": "UniProtKB:Q96GX5",
  "gene_name": "Serine_threonine-protein kinase greatwall",
  "term_id": "GO:0005634",
  "gene_symbol": "MASTL",
  "term_label": "nucleus"
}